{
  "term_id": "GO:0015271",
  "term_label": "outward rectifier potassium channel activity",
  "gene_name": "Potassium channel subfamily K member 2",
  "gene": "UniProtKB:O95069",
  "gene_symbol": "KCNK2"
}